{
  "gene": "UniProtKB:Q9H095",
  "gene_name": "Dynein regulatory complex protein 9",
  "term_id": "GO:0044782",
  "gene_symbol": "IQCG",
  "term_label": "cilium organization"
}